{
  "gene_name": "Dynein axonemal assembly factor 6",
  "gene": "UniProtKB:Q9NQM4",
  "term_label": "cytoplasm",
  "term_id": "GO:0005737",
  "gene_symbol": "DNAAF6"
}